{
  "gene": "UniProtKB:Q12809",
  "gene_symbol": "KCNH2",
  "term_id": "GO:0086091",
  "gene_name": "Potassium voltage-gated channel subfamily H member 2",
  "term_label": "regulation of heart rate by cardiac conduction"
}